{
  "term_label": "Unknown cellular component",
  "gene": "UniProtKB:Q86U02",
  "term_id": "UNKNOWN:0003",
  "gene_symbol": "LINC00596",
  "gene_name": "Putative uncharacterized protein encoded by LINC00596"
}